{
  "gene": "UniProtKB:P61289",
  "term_id": "GO:0061133",
  "gene_symbol": "PSME3",
  "term_label": "endopeptidase activator activity",
  "gene_name": "Proteasome activator complex subunit 3"
}